{
  "gene_name": "Dehydrogenase_reductase SDR family member 7B",
  "gene": "UniProtKB:Q6IAN0",
  "term_id": "UNKNOWN:0001",
  "term_label": "Unknown molecular function",
  "gene_symbol": "DHRS7B"
}